{
  "gene": "UniProtKB:Q8WWL7",
  "gene_symbol": "CCNB3",
  "term_id": "GO:0000307",
  "term_label": "cyclin-dependent protein kinase holoenzyme complex",
  "gene_name": "G2_mitotic-specific cyclin-B3"
}